blood vessel development [GO:0001568] (biological process) Definition: The process whose specific outcome is the progression of a blood vessel over time, from its formation to the mature structure. The blood vessel is the vasculature carrying blood. Sources: GOC:hjd, UBERON:0001981 Relationships: is a type of GO:0048856; is part of GO:0001944 Subtypes: placenta blood vessel development [GO:0060674], artery development [GO:0060840], venous blood vessel development [GO:0060841], coronary vasculature development [GO:0060976], glomerulus vasculature development [GO:0072012]